{
  "gene": "UniProtKB:Q9BVK8",
  "term_label": "Unknown biological process",
  "gene_symbol": "TMEM147",
  "gene_name": "BOS complex subunit TMEM147",
  "term_id": "UNKNOWN:0002"
}